{
  "gene_name": "U1 small nuclear ribonucleoprotein 70 kDa",
  "term_label": "U2-type prespliceosome",
  "gene": "UniProtKB:P08621",
  "gene_symbol": "SNRNP70",
  "term_id": "GO:0071004"
}